{
  "term_id": "GO:0015629",
  "term_label": "actin cytoskeleton",
  "gene": "UniProtKB:Q9UI15",
  "gene_name": "Transgelin-3",
  "gene_symbol": "TAGLN3"
}